{
  "gene_symbol": "DYRK2",
  "gene": "UniProtKB:Q92630",
  "term_id": "GO:0005737",
  "term_label": "cytoplasm",
  "gene_name": "Dual specificity tyrosine-phosphorylation-regulated kinase 2"
}